blastocyst development [GO:0001824] (biological process) Definition: The process whose specific outcome is the progression of the blastocyst over time, from its formation to the mature structure. The mammalian blastocyst is a hollow ball of cells containing two cell types, the inner cell mass and the trophectoderm. The blastula follows the morula and precedes the gastrula in the developmental sequence. Sources: GOC:dph, ISBN:0124020607, ISBN:0198542771 Also known as: blastula development Note: See also the Anatomical Dictionary for Mouse Development ontology terms 'TS5, embryo ; EMAP:23', 'TS5, inner cell mass ; EMAP:24' and 'TS5, trophectoderm; EMAP:28'. Relationships: is a type of anatomical structure development [GO:0048856]; is part of in utero embryonic development [GO:0001701] Regulation: RO_0002211 by regulation of blastocyst development [GO:0120222]